linoleate isomerase activity [GO:0050058] (molecular function) Definition: Catalysis of the reaction: linoleate = 9-cis,11-trans-octadecadienoate. Also known as: linoleate delta12-cis-delta11-trans-isomerase activity, linoleic acid isomerase activity Relationships: is a type of cis-trans isomerase activity [GO:0016859] Sources: EC:5.2.1.5, RHEA:17381